{
  "term_id": "UNKNOWN:0002",
  "gene_name": "Solute carrier family 35 member F2",
  "gene": "UniProtKB:Q8IXU6",
  "term_label": "Unknown biological process",
  "gene_symbol": "SLC35F2"
}